{
  "gene_name": "Target of rapamycin complex subunit LST8",
  "gene_symbol": "MLST8",
  "term_id": "GO:0031932",
  "term_label": "TORC2 complex",
  "gene": "UniProtKB:Q9BVC4"
}